{
  "gene": "UniProtKB:P37288",
  "term_label": "vasopressin receptor activity",
  "term_id": "GO:0005000",
  "gene_symbol": "AVPR1A",
  "gene_name": "Vasopressin V1a receptor"
}